{
  "term_id": "GO:0005634",
  "gene_name": "Dentin sialophosphoprotein",
  "gene": "UniProtKB:Q9NZW4",
  "gene_symbol": "DSPP",
  "term_label": "nucleus"
}